{
  "gene_name": "Mucin-like protein 1",
  "gene": "UniProtKB:Q96DR8",
  "term_id": "UNKNOWN:0002",
  "term_label": "Unknown biological process",
  "gene_symbol": "MUCL1"
}